{
  "gene_symbol": "SMAD9",
  "gene": "UniProtKB:O15198",
  "term_label": "RNA polymerase II cis-regulatory region sequence-specific DNA binding",
  "term_id": "GO:0000978",
  "gene_name": "Mothers against decapentaplegic homolog 9"
}